{
  "gene_name": "Glycerol-3-phosphate dehydrogenase [NAD(+)], cytoplasmic",
  "gene": "UniProtKB:P21695",
  "gene_symbol": "GPD1",
  "term_id": "GO:0005829",
  "term_label": "cytosol"
}